stomach body smooth muscle contraction [GO:0014845] (biological process) Relationships: is_a distal stomach smooth muscle contraction [GO:0014828] Definition: A process in which force is generated within smooth muscle tissue, resulting in a change in muscle geometry. This process occurs in the body of stomach. Force generation involves a chemo-mechanical energy conversion step that is carried out by the actin/myosin complex activity, which generates force through ATP hydrolysis. The body of stomach is the part of the stomach that lies between the fundus above and the pyloric antrum below; its boundaries are poorly defined. Sources: GOC:ef, GOC:mtg_muscle, MA:0002559